ectodermal digestive tract morphogenesis [GO:0048567] (biological process) Definition: The process in which the anatomical structures of the ectodermal digestive tract are generated and organized. The ectodermal digestive tract includes those portions of the digestive tract that are derived from ectoderm. Also known as: ectodermal gut morphogenesis Sources: GOC:jid Relationships: is a type of ectodermal digestive tract development [GO:0007439]; is part of GO:0048546